{
  "gene": "UniProtKB:P0C880",
  "gene_name": "Putative uncharacterized protein FLJ40606",
  "term_label": "Unknown molecular function",
  "term_id": "UNKNOWN:0001",
  "gene_symbol": "P0C880"
}